{
  "term_id": "GO:0000978",
  "term_label": "RNA polymerase II cis-regulatory region sequence-specific DNA binding",
  "gene": "UniProtKB:Q6PG37",
  "gene_symbol": "ZNF790",
  "gene_name": "Zinc finger protein 790"
}